{
  "gene_name": "B-cell lymphoma 3 protein",
  "term_label": "Bcl3-Bcl10 complex",
  "gene_symbol": "BCL3",
  "term_id": "GO:0032996",
  "gene": "UniProtKB:P20749"
}